{
  "gene": "UniProtKB:Q86U06",
  "gene_symbol": "RBM23",
  "gene_name": "Probable RNA-binding protein 23",
  "term_label": "Unknown cellular component",
  "term_id": "UNKNOWN:0003"
}